{
  "term_id": "GO:0002544",
  "gene_symbol": "S100A9",
  "term_label": "chronic inflammatory response",
  "gene_name": "Protein S100-A9",
  "gene": "UniProtKB:P06702"
}